{
  "term_id": "GO:0005829",
  "gene_symbol": "G6PD",
  "term_label": "cytosol",
  "gene_name": "Glucose-6-phosphate 1-dehydrogenase",
  "gene": "UniProtKB:P11413"
}